{
  "gene_name": "Ret finger protein-like 3",
  "term_label": "cytoplasm",
  "gene_symbol": "RFPL3",
  "term_id": "GO:0005737",
  "gene": "UniProtKB:O75679"
}